{
  "gene": "UniProtKB:Q15743",
  "term_id": "GO:0071467",
  "gene_name": "Ovarian cancer G-protein coupled receptor 1",
  "term_label": "cellular response to pH",
  "gene_symbol": "GPR68"
}